{
  "gene_name": "Small ribosomal subunit protein RACK1",
  "gene_symbol": "RACK1",
  "gene": "UniProtKB:P63244",
  "term_id": "GO:2001125",
  "term_label": "negative regulation of translational frameshifting"
}